{
  "gene": "UniProtKB:Q14168",
  "gene_symbol": "MPP2",
  "term_label": "Unknown biological process",
  "term_id": "UNKNOWN:0002",
  "gene_name": "MAGUK p55 subfamily member 2"
}